{
  "term_label": "Unknown cellular component",
  "gene_name": "Transmembrane protein 210",
  "gene": "UniProtKB:A6NLX4",
  "term_id": "UNKNOWN:0003",
  "gene_symbol": "TMEM210"
}